alpha-copaene biosynthetic process [GO:1901931] (biological process) Also known as: alpha-copaene anabolism, alpha-copaene biosynthesis, alpha-copaene formation, alpha-copaene synthesis References: PMID:22867794 Sources: GOC:TermGenie Definition: The chemical reactions and pathways resulting in the formation of alpha-copaene. Relationships: is a type of GO:0051762